hexitol metabolic process [GO:0006059] (BP) Subtypes: sorbitol metabolic process [GO:0006060], galactitol metabolic process [GO:0019402], hexitol biosynthetic process [GO:0019406], hexitol catabolic process [GO:0019407], mannitol metabolic process [GO:0019594] Also known as: hexitol metabolism, sugar alcohol (hexitol) metabolic process, sugar alcohol (hexitol) metabolism Sources: ISBN:0198506732 Definition: The chemical reactions and pathways involving hexitols, any alditol with a chain of six carbon atoms in the molecule. Relationships: is a type of carbohydrate metabolic process [GO:0005975]; is a type of polyol metabolic process [GO:0019751]